sesquarterpene biosynthetic process [GO:1903193] (biological process) References: PMID:21627333 Sources: GOC:TermGenie, GOC:mengo_curators, GO_REF:0000068 Definition: The chemical reactions and pathways resulting in the formation of sesquarterpene. Also known as: sesquarterpene anabolism, sesquarterpene biosynthesis, sesquarterpene formation, sesquarterpene synthesis Relationships: is a type of GO:0046246